regulation of linear element assembly [GO:0090006] (biological process) Definition: Any process that modulates the rate, frequency or extent of linear element assembly. Linear element assembly is the cell cycle process in which a proteinaceous scaffold, related to the synaptonemal complex, is assembled in association with S. pombe chromosomes during meiotic prophase. Relationships: is a type of regulation of cellular component biogenesis [GO:0044087]; is_a regulation of cellular component organization [GO:0051128]; is a type of regulation of homologous chromosome segregation [GO:0060629]; regulates GO:0030999 Sources: GOC:tb Subtypes: GO:0062123